{
  "gene_name": "Zinc finger protein 407",
  "gene_symbol": "ZNF407",
  "term_label": "transcription cis-regulatory region binding",
  "term_id": "GO:0000976",
  "gene": "UniProtKB:Q9C0G0"
}